negative regulation of basidiospore formation [GO:0075304] (BP) Definition: Any process that stops, prevents, or reduces the frequency, rate or extent of basidiospore formation, a process in which a sexually produced fungal spore is formed on a basidium in the fungi basidiomycetes. Relationships: is a type of negative regulation of sexual sporulation resulting in formation of a cellular spore [GO:0043942]; is_a GO:0075302; negatively regulates basidiospore formation [GO:0034295] Sources: GOC:pamgo_curators